{
  "gene_name": "Myotilin",
  "gene": "UniProtKB:Q9UBF9",
  "gene_symbol": "MYOT",
  "term_label": "axon guidance receptor activity",
  "term_id": "GO:0008046"
}